{
  "gene_name": "Monocarboxylate transporter 10",
  "gene_symbol": "SLC16A10",
  "term_label": "basolateral plasma membrane",
  "term_id": "GO:0016323",
  "gene": "UniProtKB:Q8TF71"
}